{
  "term_label": "Unknown biological process",
  "term_id": "UNKNOWN:0002",
  "gene_symbol": "NOS1AP",
  "gene_name": "Carboxyl-terminal PDZ ligand of neuronal nitric oxide synthase protein",
  "gene": "UniProtKB:O75052"
}